{
  "gene_name": "TBC1 domain family member 3G",
  "term_label": "Unknown cellular component",
  "gene": "UniProtKB:Q6DHY5",
  "gene_symbol": "TBC1D3G",
  "term_id": "UNKNOWN:0003"
}